neurotrophin TRK receptor binding [GO:0005167] (molecular function) Relationships: is a type of neurotrophin receptor binding [GO:0005165] Subtypes: GO:0005168, neurotrophin TRKB receptor binding [GO:0005169], GO:0005170 Also known as: neurotrophin TRK receptor ligand Definition: Binding to a neurotrophin TRK receptor. Sources: GOC:ai